{
  "gene_symbol": "GRM7",
  "gene": "UniProtKB:Q14831",
  "gene_name": "Metabotropic glutamate receptor 7",
  "term_label": "G protein-coupled glutamate receptor signaling pathway",
  "term_id": "GO:0007216"
}